smooth muscle dense body [GO:0030486] (cellular component) Definition: Electron-dense region associated with a smooth muscle contractile fiber. Sources: GOC:mah, ISBN:0815316194 Relationships: is a type of cellular anatomical structure [GO:0110165]; is part of smooth muscle contractile fiber [GO:0030485]